{
  "gene": "UniProtKB:Q9NUG6",
  "gene_name": "p53 and DNA damage-regulated protein 1",
  "term_id": "UNKNOWN:0002",
  "term_label": "Unknown biological process",
  "gene_symbol": "PDRG1"
}